 [go#goslim:chembl] Note: ChEMBL protein targets summary